{
  "gene_symbol": "CAPN9",
  "term_label": "cytoplasm",
  "gene": "UniProtKB:O14815",
  "term_id": "GO:0005737",
  "gene_name": "Calpain-9"
}